{
  "gene_name": "Protachykinin-1",
  "term_id": "GO:0005615",
  "gene": "UniProtKB:P20366",
  "term_label": "extracellular space",
  "gene_symbol": "TAC1"
}